{
  "term_label": "nucleus",
  "term_id": "GO:0005634",
  "gene_name": "Sodium channel modifier 1",
  "gene": "UniProtKB:Q9BWG6",
  "gene_symbol": "SCNM1"
}